{
  "term_label": "glycerol kinase activity",
  "gene_name": "Putative glycerol kinase 5",
  "gene_symbol": "GK5",
  "term_id": "GO:0004370",
  "gene": "UniProtKB:Q6ZS86"
}